{
  "gene_name": "NF-kappa-B essential modulator",
  "term_id": "GO:0043123",
  "gene": "UniProtKB:Q9Y6K9",
  "term_label": "positive regulation of canonical NF-kappaB signal transduction",
  "gene_symbol": "IKBKG"
}